negative regulation of translation in response to endoplasmic reticulum stress [GO:1902010] (biological process) Definition: Any process that stops, prevents, or reduces the frequency, rate or extent of translation as a result of endoplasmic reticulum stress. References: PMID:10882126 Sources: GOC:TermGenie, GOC:dph Also known as: down regulation of protein biosynthetic process involved in ER stress response, down regulation of protein biosynthetic process involved in response to ER stress, down regulation of protein biosynthetic process involved in response to endoplasmic reticulum stress, down-regulation of protein biosynthetic process involved in ER stress response, down-regulation of protein biosynthetic process involved in response to ER stress, down-regulation of protein biosynthetic process involved in response to endoplasmic reticulum stress, downregulation of protein biosynthetic process involved in ER stress response, downregulation of protein biosynthetic process involved in response to ER stress, downregulation of protein biosynthetic process involved in response to endoplasmic reticulum stress, negative regulation of protein anabolism involved in ER stress response, negative regulation of protein anabolism involved in response to ER stress, negative regulation of protein anabolism involved in response to endoplasmic reticulum stress, negative regulation of protein biosynthesis involved in ER stress response, negative regulation of protein biosynthesis involved in response to ER stress, negative regulation of protein biosynthesis involved in response to endoplasmic reticulum stress, negative regulation of protein biosynthetic process involved in ER stress response, negative regulation of protein biosynthetic process involved in response to ER stress, negative regulation of protein biosynthetic process involved in response to endoplasmic reticulum stress, negative regulation of protein formation involved in ER stress response, negative regulation of protein formation involved in response to ER stress, negative regulation of protein formation involved in response to endoplasmic reticulum stress, negative regulation of protein synthesis involved in ER stress response, negative regulation of protein synthesis involved in response to ER stress, negative regulation of protein synthesis involved in response to endoplasmic reticulum stress, negative regulation of translation involved in ER stress response, negative regulation of translation involved in response to ER stress, inhibition of protein biosynthetic process involved in ER stress response, inhibition of protein biosynthetic process involved in response to ER stress, inhibition of protein biosynthetic process involved in response to endoplasmic reticulum stress, protein biosynthesis inhibitor activity involved in ER stress response, protein biosynthesis inhibitor activity involved in response to ER stress, protein biosynthesis inhibitor activity involved in response to endoplasmic reticulum stress, protein biosynthetic process inhibitor activity involved in ER stress response, protein biosynthetic process inhibitor activity involved in response to ER stress, protein biosynthetic process inhibitor activity involved in response to endoplasmic reticulum stress Relationships: is_a negative regulation of translation in response to stress [GO:0032055]; is a type of regulation of translation in response to endoplasmic reticulum stress [GO:0036490] Subtypes: negative regulation of translation initiation in response to endoplasmic reticulum stress [GO:0036495]